{
  "gene_name": "Plastin-3",
  "term_label": "actin filament network formation",
  "gene_symbol": "PLS3",
  "term_id": "GO:0051639",
  "gene": "UniProtKB:P13797"
}